reproductive behavior [GO:0019098] (biological process) Definition: The specific behavior of an organism that is associated with reproduction. Also known as: reproductive behavior in a multicellular organism, reproductive behaviour, multi-organism reproductive behavior, multicellular organism reproductive behavior, single-organism reproductive behavior Sources: GOC:jl, GOC:pr Subtypes: mating behavior [GO:0007617], GO:0018991, parental behavior [GO:0060746] Relationships: is a type of GO:0007610; is_a multicellular organismal reproductive process [GO:0048609]